{
  "gene_name": "Serine_arginine repetitive matrix protein 3",
  "term_id": "UNKNOWN:0003",
  "term_label": "Unknown cellular component",
  "gene": "UniProtKB:A6NNA2",
  "gene_symbol": "SRRM3"
}